L-methionine transmembrane transporter activity [GO:0015191] (molecular function) Relationships: is a type of L-amino acid transmembrane transporter activity [GO:0015179]; is a type of methionine transmembrane transporter activity [GO:0043865] Definition: Enables the transfer of L-methionine from one side of a membrane to the other. L-methionine is 2-amino-4-(methylthio)butanoic acid. Sources: GOC:ai, GOC:mtg_transport, ISBN:0815340729 Also known as: L-methionine transporter activity Subtypes: GO:0000102